6a-hydroxymaackiain-3-O-methyltransferase activity [GO:0102671] (molecular function) Definition: Catalysis of the reaction: (+)-6a-hydroxymaackiain + S-adenosyl-L-methionine = H+ + (+)-pisatin + S-adenosyl-L-homocysteine. Relationships: is a type of methyltransferase activity [GO:0008168] Sources: EC:2.1.1.270, GOC:pz